symbiont-mediated evasion of recognition by host antimicrobial peptide [GO:0141179] (biological process) Definition: A process by which a symbiont avoids the effects of recognition by a host  antimicrobial peptide by altering molecules on the symbiont surface. The host is defined as the larger of the organisms involved in a symbiotic interaction. Relationships: is a type of symbiont-mediated evasion of recognition by host innate immune effector [GO:0141177] References: PMID:11401964, PMID:22966934, PMID:25537831